{
  "gene_symbol": "MUSTN1",
  "term_label": "Unknown biological process",
  "term_id": "UNKNOWN:0002",
  "gene_name": "Musculoskeletal embryonic nuclear protein 1",
  "gene": "UniProtKB:Q8IVN3"
}